{
  "gene_name": "Protein shisa-6",
  "term_label": "AMPA glutamate receptor complex",
  "gene": "UniProtKB:Q6ZSJ9",
  "term_id": "GO:0032281",
  "gene_symbol": "SHISA6"
}